{
  "term_id": "GO:0000978",
  "term_label": "RNA polymerase II cis-regulatory region sequence-specific DNA binding",
  "gene_symbol": "ZBTB41",
  "gene": "UniProtKB:Q5SVQ8",
  "gene_name": "Zinc finger and BTB domain-containing protein 41"
}